regulation of formation of translation preinitiation complex [GO:1901193] (biological process) Definition: Any process that modulates the frequency, rate or extent of formation of translation preinitiation complex. Relationships: is a type of regulation of protein-containing complex assembly [GO:0043254]; is a type of regulation of cytoplasmic translational initiation [GO:1904688]; regulates formation of translation preinitiation complex [GO:0001731] Sources: GOC:TermGenie Also known as: regulation of formation of translation pre-initiation complex, regulation of translation preinitiation complex assembly Subtypes: negative regulation of formation of translation preinitiation complex [GO:1901194], positive regulation of formation of translation preinitiation complex [GO:1901195]